{
  "gene_name": "Immunoglobulin-like domain-containing receptor 2",
  "term_label": "membrane",
  "gene_symbol": "ILDR2",
  "term_id": "GO:0016020",
  "gene": "UniProtKB:Q71H61"
}